P-type monovalent copper transporter activity [GO:0140581] (molecular function) Sources: RHEA:25792 Definition: Enables the transfer of a solute or solutes from one side of a membrane to the other according to the reaction: ATP + H2O + Cu+(in) = ADP + phosphate + Cu+(out). Relationships: is a type of GO:0005375; is a type of P-type ion transporter activity [GO:0015662]; is a type of ATPase-coupled monoatomic cation transmembrane transporter activity [GO:0019829] Note: Note that this enzyme transports Cu(+) or Ag(+), and cannot transport the divalent ions, contrary to EC:7.2.2.9, which mainly transports the divalent copper ion (source: EC:7.2.2.8).